{
  "gene_name": "Protein transport protein Sec24D",
  "term_id": "GO:0008270",
  "gene_symbol": "SEC24D",
  "term_label": "zinc ion binding",
  "gene": "UniProtKB:O94855"
}